{
  "term_label": "Unknown cellular component",
  "term_id": "UNKNOWN:0003",
  "gene_symbol": "ZMAT1",
  "gene": "UniProtKB:Q5H9K5",
  "gene_name": "Zinc finger matrin-type protein 1"
}